6-O-methylnorlaudanosoline 5'-O-methyltransferase activity [GO:0030781] (molecular function) Sources: EC:2.1.1.121 Also known as: S-adenosyl-L-methionine:6-O-methylnorlaudanosoline 5'-O-methyltransferase activity Definition: Catalysis of the reaction: S-adenosyl-L-methionine + 6-O-methylnorlaudanosoline = S-adenosyl-L-homocysteine + nororientaline. Relationships: is a type of S-adenosylmethionine-dependent methyltransferase activity [GO:0008757]